cleavage between 5.8S rRNA and 2S rRNA of tetracistronic rRNA transcript (SSU-rRNA, 5.8S rRNA, 2S rRNA, LSU-rRNA) [GO:0000486] (biological process) Relationships: is a type of endonucleolytic cleavage of tetracistronic rRNA transcript (SSU-rRNA, 5.8S rRNA, 2S rRNA, LSU-rRNA) [GO:0000483]; BFO_0000050 maturation of 2S rRNA [GO:0000475]; is part of GO:0000487 Definition: Endonucleolytic cleavage between the 5.8S rRNA and the 2S rRNA of an rRNA molecule originally produced as a tetracistronic rRNA transcript that contained the Small SubUnit (SSU) rRNA, the 5.8S rRNA, 2S rRNA, and the Large SubUnit (LSU) rRNA, in that order, from 5' to 3' along the primary transcript. References: PMID:768488 Sources: GOC:curators